{
  "term_id": "GO:0110104",
  "gene_symbol": "CPSF7",
  "gene": "UniProtKB:Q8N684",
  "term_label": "mRNA alternative polyadenylation",
  "gene_name": "Cleavage and polyadenylation specificity factor subunit 7"
}